{
  "gene_symbol": "CD93",
  "gene": "UniProtKB:Q9NPY3",
  "term_id": "GO:0038023",
  "term_label": "signaling receptor activity",
  "gene_name": "Complement component C1q receptor"
}